{
  "term_label": "synapse",
  "gene_symbol": "CNTNAP5",
  "gene_name": "Contactin-associated protein-like 5",
  "term_id": "GO:0045202",
  "gene": "UniProtKB:Q8WYK1"
}